delayed rectifier potassium channel activity [GO:0005251] (molecular function) Regulation: regulated by GO:1902259; negatively regulated by negative regulation of delayed rectifier potassium channel activity [GO:1902260] References: PMID:11343411, PMID:2462513 Sources: GOC:mah Relationships: is a type of voltage-gated potassium channel activity [GO:0005249] Definition: Enables the transmembrane transfer of a potassium ion by a delayed rectifying voltage-gated channel. A delayed rectifying current-voltage relation is one where channel activation kinetics are time-dependent, and inactivation is slow.